{
  "gene": "UniProtKB:Q9Y228",
  "gene_symbol": "TRAF3IP3",
  "term_label": "molecular adaptor activity",
  "term_id": "GO:0060090",
  "gene_name": "TRAF3-interacting JNK-activating modulator"
}